nucleotide transmembrane transport [GO:1901679] (biological process) Definition: The directed movement of nucleotide across a membrane. Sources: GOC:TermGenie, GOC:pr Also known as: nucleotide membrane transport Note: Note that this term is not intended for use in annotating lateral movement within membranes. Relationships: is a type of nucleotide transport [GO:0006862]; is a type of transmembrane transport [GO:0055085] Subtypes: FAD transmembrane transport [GO:0035350], NAD transmembrane transport [GO:0035352], nicotinamide mononucleotide transmembrane transport [GO:0035353], GO:0071106, mitochondrial ADP transmembrane transport [GO:0140021], 5'-adenylyl sulfate transmembrane transport [GO:1902558], 3'-phospho-5'-adenylyl sulfate transmembrane transport [GO:1902559], guanine nucleotide transmembrane transport [GO:1903790], GO:1990519, mitochondrial ATP transmembrane transport [GO:1990544]